{
  "gene_name": "Leucine-rich colipase-like protein 1",
  "term_label": "Unknown cellular component",
  "term_id": "UNKNOWN:0003",
  "gene_symbol": "LRCOL1",
  "gene": "UniProtKB:A6NCL2"
}